{
  "term_id": "GO:0071805",
  "term_label": "potassium ion transmembrane transport",
  "gene": "UniProtKB:Q9NR82",
  "gene_symbol": "KCNQ5",
  "gene_name": "Potassium voltage-gated channel subfamily KQT member 5"
}